alcohol O-acetyltransferase activity [GO:0004026] (MF) Definition: Catalysis of the reaction: acetyl-CoA + an alcohol = CoA + an acetyl ester. Also known as: AATASE activity, acetyl-CoA:alcohol O-acetyltransferase activity, alcohol acetyltransferase activity Relationships: is a type of O-acetyltransferase activity [GO:0016413]; is_a alcohol O-acyltransferase activity [GO:0034318] Sources: EC:2.3.1.84